pyrrolysine biosynthetic process [GO:0071524] (biological process) Definition: The chemical reactions and pathways resulting in the formation of pyrrolysine, N6-{[(2R,3R)-3-methyl-3,4-dihydro-2H-pyrrol-2-yl]carbonyl}-L-lysine. References: PMID:17204561 Sources: GOC:dh Relationships: is a type of amino acid biosynthetic process [GO:0008652]; is a type of modified amino acid biosynthetic process [GO:0042398]; is a type of amide biosynthetic process [GO:0043604]; is a type of GO:0170038 Also known as: monomethylamine methyltransferase cofactor lysine adduct biosynthetic process, pyrrolysine anabolism, pyrrolysine biosynthesis, pyrrolysine formation, pyrrolysine synthesis